{
  "term_id": "UNKNOWN:0003",
  "gene_symbol": "TRGV10",
  "gene_name": "Probable non-functional T cell receptor gamma variable 10",
  "gene": "UniProtKB:A0A0A0MS01",
  "term_label": "Unknown cellular component"
}